{
  "gene_name": "SPARC-related modular calcium-binding protein 2",
  "gene_symbol": "SMOC2",
  "gene": "UniProtKB:Q9H3U7",
  "term_label": "extracellular matrix binding",
  "term_id": "GO:0050840"
}